{
  "gene_name": "cAMP-dependent protein kinase catalytic subunit gamma",
  "term_label": "cAMP-dependent protein kinase complex",
  "gene_symbol": "PRKACG",
  "gene": "UniProtKB:P22612",
  "term_id": "GO:0005952"
}